{
  "gene_name": "Platelet-activating factor acetylhydrolase IB subunit alpha1",
  "gene": "UniProtKB:Q15102",
  "gene_symbol": "PAFAH1B3",
  "term_id": "GO:0003847",
  "term_label": "1-alkyl-2-acetylglycerophosphocholine esterase activity"
}